positive regulation of muscle cell differentiation [GO:0051149] (biological process) Definition: Any process that activates or increases the frequency, rate or extent of muscle cell differentiation. Subtypes: positive regulation of smooth muscle cell differentiation [GO:0051152], positive regulation of striated muscle cell differentiation [GO:0051155] Sources: CL:0000187, GOC:ai Also known as: up regulation of muscle cell differentiation, up-regulation of muscle cell differentiation, upregulation of muscle cell differentiation, activation of muscle cell differentiation, stimulation of muscle cell differentiation Relationships: is a type of positive regulation of cell differentiation [GO:0045597]; is a type of regulation of muscle cell differentiation [GO:0051147]; positively regulates muscle cell differentiation [GO:0042692]